{
  "term_label": "intracellular protein localization",
  "gene": "UniProtKB:O43572",
  "gene_symbol": "AKAP10",
  "term_id": "GO:0008104",
  "gene_name": "A-kinase anchor protein 10, mitochondrial"
}